{
  "term_id": "GO:0043490",
  "term_label": "malate-aspartate shuttle",
  "gene": "UniProtKB:Q9UJS0",
  "gene_symbol": "SLC25A13",
  "gene_name": "Electrogenic aspartate_glutamate antiporter SLC25A13, mitochondrial"
}